{
  "gene_symbol": "CHRNB2",
  "gene": "UniProtKB:P17787",
  "term_id": "GO:0015464",
  "gene_name": "Neuronal acetylcholine receptor subunit beta-2",
  "term_label": "acetylcholine receptor activity"
}